protein-glutamate O-methyltransferase activity [GO:0008983] (molecular function) Definition: Catalysis of the reaction: S-adenosyl-L-methionine + protein L-glutamate = S-adenosyl-L-homocysteine + protein L-glutamate 5-methyl ester; this reaction is the methylation of peptidyl-L-glutamate to form peptidyl-L-glutamate 5-methyl ester. Sources: EC:2.1.1.80 Also known as: protein glutamate O-methylase activity, protein glutamate O-methyltransferase activity, methyl-accepting chemotaxis protein O-methyltransferase activity, MCP methyltransferase I, MCP methyltransferase II, S-adenosyl-L-methionine:protein-L-glutamate O-methyltransferase activity, S-adenosylmethionine-glutamyl methyltransferase activity, S-adenosylmethionine:protein-carboxyl O-methyltransferase activity, methyl-accepting chemotaxis protein methyltransferase II, protein O-methyltransferase activity, protein carboxyl-O-methyltransferase activity, protein carboxyl-methylase activity, protein carboxylmethyltransferase II, protein carboxymethylase activity, protein carboxymethyltransferase activity, protein methylase II, protein(aspartate)methyltransferase activity, protein(carboxyl)methyltransferase activity Relationships: is_a S-adenosylmethionine-dependent methyltransferase activity [GO:0008757]; is a type of protein carboxyl O-methyltransferase activity [GO:0051998]